{
  "gene": "UniProtKB:Q9NX63",
  "gene_name": "MICOS complex subunit MIC19",
  "gene_symbol": "CHCHD3",
  "term_id": "GO:0007007",
  "term_label": "inner mitochondrial membrane organization"
}